voluntary musculoskeletal movement [GO:0050882] (biological process) Sources: GOC:dph Relationships: is a type of GO:0050881 Definition: The movement of an organism or part of an organism using mechanoreceptors, the nervous system, striated muscle and/or the skeletal system that can be controlled at will.